LRR domain binding [GO:0030275] (molecular function) Sources: GOC:go_curators, Pfam:PF00560 Subtypes: leucine zipper domain binding [GO:0043522] Definition: Binding to a LRR domain (leucine rich repeats) of a protein. Relationships: is a type of protein domain specific binding [GO:0019904]